negative regulation of cytotoxic T cell differentiation [GO:0045584] (biological process) Also known as: down regulation of cytotoxic T cell differentiation, down-regulation of cytotoxic T cell differentiation, downregulation of cytotoxic T cell differentiation, negative regulation of cytotoxic T lymphocyte differentiation, negative regulation of cytotoxic T-cell differentiation, negative regulation of cytotoxic T-lymphocyte differentiation, inhibition of cytotoxic T cell differentiation, negative regulation of cytotoxic T cell development Definition: Any process that stops, prevents, or reduces the frequency, rate or extent of cytotoxic T cell differentiation. Relationships: is a type of negative regulation of T cell differentiation [GO:0045581]; is a type of regulation of cytotoxic T cell differentiation [GO:0045583]; negatively regulates cytotoxic T cell differentiation [GO:0045065] Note: Note that immunologists typically use the word 'development' to refer to cells of B or T cell lineages undergoing the process that GO describes as 'cell differentiation'. Sources: GOC:go_curators